{
  "gene": "UniProtKB:Q9ULC0",
  "term_label": "Unknown cellular component",
  "gene_symbol": "EMCN",
  "term_id": "UNKNOWN:0003",
  "gene_name": "Endomucin"
}